{
  "term_id": "GO:0099558",
  "gene_symbol": "C1QL3",
  "gene": "UniProtKB:Q5VWW1",
  "term_label": "maintenance of synapse structure",
  "gene_name": "Complement C1q-like protein 3"
}